{
  "gene": "UniProtKB:Q9NYA3",
  "term_id": "UNKNOWN:0001",
  "term_label": "Unknown molecular function",
  "gene_name": "Golgin subfamily A member 6A",
  "gene_symbol": "GOLGA6A"
}